{
  "gene_name": "Synaptotagmin-17",
  "term_label": "regulation of calcium ion-dependent exocytosis",
  "term_id": "GO:0017158",
  "gene": "UniProtKB:Q9BSW7",
  "gene_symbol": "SYT17"
}